uniporter activity [GO:0015292] (molecular function) Subtypes: GO:0008516, phenyl propionate uniporter activity [GO:0015544], membrane potential driven uniporter activity [GO:0022810], dipeptide uniporter activity [GO:0160178] Relationships: is a type of secondary active transmembrane transporter activity [GO:0015291] Also known as: facilitated diffusion carrier, single-species transporter activity, uniport Definition: Catalysis of the transport of a single molecular species across a membrane; transport is independent of the movement of any other molecular species. References: PMID:10839820 Sources: GOC:mtg_transport, ISBN:0815340729